{
  "gene_name": "Endogenous retrovirus group K3 member 1",
  "term_label": "Unknown molecular function",
  "gene": "UniProtKB:B3KNS4",
  "term_id": "UNKNOWN:0001",
  "gene_symbol": "ERVK3-1"
}